{
  "gene_symbol": "IGHJ2",
  "gene_name": "Immunoglobulin heavy joining 2 (Fragment)",
  "term_id": "UNKNOWN:0001",
  "gene": "UniProtKB:A0A0J9YWN2",
  "term_label": "Unknown molecular function"
}